{
  "gene_symbol": "KRTAP7-1",
  "gene": "UniProtKB:Q8IUC3",
  "gene_name": "Keratin-associated protein 7-1",
  "term_label": "Unknown molecular function",
  "term_id": "UNKNOWN:0001"
}